general transcription initiation factor binding [GO:0140296] (molecular function) Relationships: is a type of transcription factor binding [GO:0008134] Sources: GOC:txnOH-2018 Definition: Binding to a general transcription initiation factor, a protein that contributes to transcription start site selection and transcription initiation. Subtypes: GO:0001025, GO:0001091, RNA polymerase I general transcription initiation factor binding [GO:0001179], TBP-class protein binding [GO:0017025]